{
  "gene_name": "Probable inactive ribonuclease-like protein 13",
  "gene": "UniProtKB:Q5GAN3",
  "gene_symbol": "RNASE13",
  "term_label": "Unknown cellular component",
  "term_id": "UNKNOWN:0003"
}